{
  "term_id": "UNKNOWN:0001",
  "gene": "UniProtKB:O00631",
  "gene_symbol": "SLN",
  "gene_name": "Sarcolipin",
  "term_label": "Unknown molecular function"
}